{
  "term_label": "fatty acid beta-oxidation",
  "gene_name": "Peroxisomal multifunctional enzyme type 2",
  "gene": "UniProtKB:P51659",
  "term_id": "GO:0006635",
  "gene_symbol": "HSD17B4"
}